{
  "term_label": "ubiquitin-dependent protein catabolic process",
  "gene_name": "Ubiquitin-conjugating enzyme E2 D2",
  "term_id": "GO:0006511",
  "gene_symbol": "UBE2D2",
  "gene": "UniProtKB:P62837"
}